{
  "gene": "UniProtKB:Q9Y3S1",
  "gene_symbol": "WNK2",
  "gene_name": "Serine_threonine-protein kinase WNK2",
  "term_id": "GO:0005829",
  "term_label": "cytosol"
}